{
  "gene_name": "Transmembrane protein 266",
  "gene_symbol": "TMEM266",
  "term_label": "dendrite",
  "term_id": "GO:0030425",
  "gene": "UniProtKB:Q2M3C6"
}